{
  "gene_symbol": "SLC2A13",
  "gene": "UniProtKB:Q96QE2",
  "term_label": "apical plasma membrane",
  "gene_name": "Proton myo-inositol cotransporter",
  "term_id": "GO:0016324"
}